{
  "gene": "UniProtKB:Q8NBJ4",
  "term_label": "Unknown molecular function",
  "term_id": "UNKNOWN:0001",
  "gene_symbol": "GOLM1",
  "gene_name": "Golgi membrane protein 1"
}